regulation of mesonephric nephron tubule epithelial cell differentiation [GO:2000093] (biological process) Definition: Any process that modulates the frequency, rate or extent of mesonephric nephron tubule epithelial cell differentiation. Relationships: is a type of regulation of nephron tubule epithelial cell differentiation [GO:0072182]; regulates GO:0061265 Sources: GOC:mtg_kidney_jan10 Subtypes: negative regulation of mesonephric nephron tubule epithelial cell differentiation [GO:2000094]